{
  "gene_name": "RAB6-interacting golgin",
  "term_id": "GO:1905515",
  "gene": "UniProtKB:Q5T7V8",
  "term_label": "non-motile cilium assembly",
  "gene_symbol": "GORAB"
}